{
  "gene_name": "Doublecortin domain-containing protein 2C",
  "gene_symbol": "DCDC2C",
  "gene": "UniProtKB:A8MYV0",
  "term_id": "UNKNOWN:0002",
  "term_label": "Unknown biological process"
}